{
  "gene_name": "DNA-binding death effector domain-containing protein 2",
  "term_label": "extrinsic apoptotic signaling pathway via death domain receptors",
  "gene": "UniProtKB:Q8WXF8",
  "gene_symbol": "DEDD2",
  "term_id": "GO:0008625"
}